{
  "gene": "UniProtKB:P18065",
  "term_label": "regulation of insulin-like growth factor receptor signaling pathway",
  "term_id": "GO:0043567",
  "gene_name": "Insulin-like growth factor-binding protein 2",
  "gene_symbol": "IGFBP2"
}